{
  "term_label": "glucosamine catabolic process",
  "term_id": "GO:0006043",
  "gene_symbol": "GNPDA1",
  "gene": "UniProtKB:P46926",
  "gene_name": "Glucosamine-6-phosphate isomerase 1"
}